{
  "term_label": "cytoplasmic side of plasma membrane",
  "gene_symbol": "CHMP4BP1",
  "term_id": "GO:0009898",
  "gene_name": "Putative charged multivesicular body protein 4B-like protein CHMP4BP1",
  "gene": "UniProtKB:P59074"
}